{
  "gene_symbol": "BOK",
  "gene_name": "Bcl-2-related ovarian killer protein",
  "term_id": "GO:0001836",
  "term_label": "release of cytochrome c from mitochondria",
  "gene": "UniProtKB:Q9UMX3"
}